{
  "gene": "UniProtKB:Q5VWX1",
  "term_label": "regulation of alternative mRNA splicing, via spliceosome",
  "gene_symbol": "KHDRBS2",
  "term_id": "GO:0000381",
  "gene_name": "KH domain-containing, RNA-binding, signal transduction-associated protein 2"
}